{
  "term_label": "transcription elongation-coupled chromatin remodeling",
  "term_id": "GO:0140673",
  "gene_symbol": "USP15",
  "gene_name": "Ubiquitin carboxyl-terminal hydrolase 15",
  "gene": "UniProtKB:Q9Y4E8"
}